cellular response to magnesium ion [GO:0071286] (biological process) Sources: GOC:mah Relationships: is a type of response to magnesium ion [GO:0032026]; is a type of cellular response to metal ion [GO:0071248] Definition: Any process that results in a change in state or activity of a cell (in terms of movement, secretion, enzyme production, gene expression, etc.) as a result of a magnesium ion stimulus.